{
  "term_id": "GO:0042438",
  "gene_name": "Melanocyte-stimulating hormone receptor",
  "term_label": "melanin biosynthetic process",
  "gene_symbol": "MC1R",
  "gene": "UniProtKB:Q01726"
}